cilium-dependent cell motility [GO:0060285] (biological process) Sources: GOC:cilia, GOC:dgh, GOC:dph, GOC:krc, GOC:mlg Definition: Cell motility due to the motion of one or more eukaryotic cilia. A eukaryotic cilium is a specialized organelle that consists of a filiform extrusion of the cell surface. Each cilium is bounded by an extrusion of the cytoplasmic (plasma) membrane, and contains a regular longitudinal array of microtubules, anchored basally in a centriole. Also known as: cilium cell motility, microtubule-based flagellar cell motility, ciliary cell motility Regulation: regulated by regulation of cilium-dependent cell motility [GO:1902019]; negatively regulated by negative regulation of cilium-dependent cell motility [GO:1902020]; RO_0002213 by positive regulation of cilium-dependent cell motility [GO:2000155] Relationships: is a type of cilium or flagellum-dependent cell motility [GO:0001539]; has part cilium movement [GO:0003341] Subtypes: flagellated sperm motility [GO:0030317] Note: Note that we deem eukaryotic cilia and microtubule-based flagella to be equivalent.